'de novo' NAD+ biosynthetic process from L-aspartate [GO:0034628] (biological process) Note: This pathway is found in bacteria, Archaea and may also occur in plants. Relationships: is a type of GO:0006531; is a type of GO:0009435; is a type of L-amino acid metabolic process [GO:0170033]; is a type of proteinogenic amino acid metabolic process [GO:0170039] Also known as: 'de novo' NAD biosynthetic process from aspartate, 'de novo' NAD biosynthetic process from L-aspartate, nicotinamide nucleotide anabolism from aspartate, nicotinamide nucleotide biosynthetic process from aspartate, nicotinamide nucleotide formation from aspartate, nicotinamide nucleotide synthesis from aspartate, de novo NAD biosynthetic process from aspartate Definition: The chemical reactions and pathways resulting in the formation of nicotinamide adenine dinucleotide (NAD+), beginning with the catabolism of L-aspartate into the precursor quinolinate. NAD+ is a coenzyme that interconverts with its reduced form, NADH, in many redox and catabolic reactions. Sources: GOC:curators